ribonucleoside bisphosphate catabolic process [GO:0034031] (biological process) Sources: GOC:mah, GOC:pde Also known as: ribonucleoside bisphosphate breakdown, ribonucleoside bisphosphate catabolism, ribonucleoside bisphosphate degradation Subtypes: purine ribonucleoside bisphosphate catabolic process [GO:0034037] Definition: The chemical reactions and pathways resulting in the breakdown of a ribonucleoside bisphosphate, a compound consisting of a nucleobase linked to a ribose sugar esterified with one phosphate group attached to each of two different hydroxyl groups on the sugar. Relationships: is a type of nucleoside bisphosphate catabolic process [GO:0033869]; is a type of GO:0033875